peptidyl-proline hydroxylation to 4-hydroxy-L-proline [GO:0018401] (biological process) Relationships: is a type of modified amino acid metabolic process [GO:0006575]; is a type of GO:0019511; is a type of GO:0170033; is a type of non-proteinogenic amino acid metabolic process [GO:0170041] Definition: The modification of peptidyl-proline to form 4-hydroxy-L-proline; catalyzed by procollagen-proline,2-oxoglutarate-4-dioxygenase. Sources: RESID:AA0030 Note: See also the molecular function term 'procollagen-proline 4-dioxygenase activity ; GO:0004656'.